{
  "gene_name": "ATM interactor",
  "term_id": "GO:0000976",
  "gene_symbol": "ATMIN",
  "term_label": "transcription cis-regulatory region binding",
  "gene": "UniProtKB:O43313"
}